precorrin-4 C11-methyltransferase activity [GO:0046026] (molecular function) Also known as: CobM, S-adenosyl-L-methionine:precorrin-4 C11 methyltransferase activity Relationships: is a type of S-adenosylmethionine-dependent methyltransferase activity [GO:0008757] Sources: EC:2.1.1.133 Definition: Catalysis of the reaction: S-adenosyl-L-methionine + precorrin-4 = S-adenosyl-L-homocysteine + precorrin 5.